{
  "gene": "UniProtKB:Q9UBP4",
  "term_label": "extracellular space",
  "gene_symbol": "DKK3",
  "term_id": "GO:0005615",
  "gene_name": "Dickkopf-related protein 3"
}